{
  "term_id": "GO:0042391",
  "term_label": "regulation of membrane potential",
  "gene_symbol": "PIEZO2",
  "gene": "UniProtKB:Q9H5I5",
  "gene_name": "Piezo-type mechanosensitive ion channel component 2"
}